regulation of type II interferon production [GO:0032649] (biological process) Relationships: is a type of regulation of cytokine production [GO:0001817]; regulates type II interferon production [GO:0032609] References: PMID:15546383 Sources: GOC:add, GOC:mah Definition: Any process that modulates the frequency, rate, or extent of interferon-gamma production. Interferon-gamma is also known as type II interferon. Subtypes: negative regulation of type II interferon production [GO:0032689], positive regulation of type II interferon production [GO:0032729] Also known as: regulation of interferon-gamma production, regulation of interferon-gamma biosynthetic process, regulation of interferon-gamma secretion